{
  "term_id": "UNKNOWN:0003",
  "term_label": "Unknown cellular component",
  "gene": "UniProtKB:Q96PX6",
  "gene_name": "Coiled-coil domain-containing protein 85A",
  "gene_symbol": "CCDC85A"
}